{
  "gene_symbol": "SDHAF3",
  "term_label": "Unknown molecular function",
  "gene": "UniProtKB:Q9NRP4",
  "gene_name": "Succinate dehydrogenase assembly factor 3, mitochondrial",
  "term_id": "UNKNOWN:0001"
}